photoreceptor disc membrane [GO:0097381] (cellular component) References: PMID:11826267, PMID:19501669, PMID:2537204, PMID:26574505, PMID:6771304, PMID:7507907 Sources: GOC:bj, GOC:krc, GOC:pde Relationships: is a type of organelle membrane [GO:0031090]; is part of GO:0001750 Definition: Stack of disc membranes located inside a photoreceptor outer segment, and containing densely packed molecules of photoreceptor proteins that traverse the lipid bilayer. Disc membranes arise as evaginations of the ciliary membrane during the development of the outer segment and may or may not remain contiguous with the ciliary membrane. Subtypes: cone photoreceptor disc membrane [GO:0120201], rod photoreceptor disc membrane [GO:0120202]